{
  "gene_name": "Zinc finger protein 703",
  "term_id": "GO:0005634",
  "gene": "UniProtKB:Q9H7S9",
  "gene_symbol": "ZNF703",
  "term_label": "nucleus"
}